diol biosynthetic process [GO:0034312] (biological process) Definition: The chemical reactions and pathways resulting in the formation of a diol, any alcohol containing two hydroxyl groups attached to saturated carbon atoms. Sources: GOC:mah Subtypes: GO:0006729, glycol biosynthetic process [GO:0042845], sphinganine biosynthetic process [GO:0046511], sphingosine biosynthetic process [GO:0046512], GO:0106210, asperfuranone biosynthetic process [GO:1900554], GO:1902135, (-)-secoisolariciresinol biosynthetic process [GO:1902138], verruculogen biosynthetic process [GO:1902181] Also known as: dihydric alcohol biosynthetic process, diol anabolism, diol biosynthesis, diol formation, diol synthesis Relationships: is_a diol metabolic process [GO:0034311]; is a type of GO:0046173